{
  "term_label": "endocytosis",
  "term_id": "GO:0006897",
  "gene": "UniProtKB:Q13636",
  "gene_symbol": "RAB31",
  "gene_name": "Ras-related protein Rab-31"
}